dentate nucleus development [GO:0021735] (biological process) Definition: The process whose specific outcome is the progression of the dentate nucleus over time, from its formation to the mature structure. Relationships: is a type of neural nucleus development [GO:0048857]; is part of cerebellum development [GO:0021549] Sources: GOC:cls, GOC:curators, GOC:dgh, GOC:dph, GOC:jid